{
  "term_label": "mRNA splicing, via spliceosome",
  "gene": "UniProtKB:P62306",
  "term_id": "GO:0000398",
  "gene_name": "Small nuclear ribonucleoprotein F",
  "gene_symbol": "SNRPF"
}